{
  "term_id": "GO:0002682",
  "gene_symbol": "ZBTB12",
  "gene": "UniProtKB:Q9Y330",
  "term_label": "regulation of immune system process",
  "gene_name": "Zinc finger and BTB domain-containing protein 12"
}